non-motile cilium [GO:0097730] (cellular component) Definition: A cilium which may have a variable array of axonemal microtubules but does not contain molecular motors. References: PMID:17009929, PMID:20144998, PMID:22118931 Sources: GOC:cilia, GOC:dgh, GOC:kmv Also known as: immotile cilium, nonmotile cilium, immotile primary cilium, nonmotile primary cilia, nonmotile primary cilium, sensory cilium Relationships: is a type of cilium [GO:0005929] Subtypes: 9+0 non-motile cilium [GO:0097731], 9+2 non-motile cilium [GO:0097732]